{
  "gene": "UniProtKB:Q03181",
  "term_label": "positive regulation of fatty acid metabolic process",
  "gene_symbol": "PPARD",
  "term_id": "GO:0045923",
  "gene_name": "Peroxisome proliferator-activated receptor delta"
}